U6 snRNA 3'-end processing [GO:0034477] (biological process) Relationships: is a type of GO:0034472 Sources: GOC:mah Also known as: U6 snRNA 3' end processing Definition: Any process involved in forming the mature 3' end of a U6 snRNA molecule.